{
  "term_id": "GO:0030154",
  "term_label": "cell differentiation",
  "gene_name": "Protein C-ets-1",
  "gene_symbol": "ETS1",
  "gene": "UniProtKB:P14921"
}